{
  "gene": "UniProtKB:Q9P2K1",
  "term_label": "protein localization to ciliary transition zone",
  "gene_symbol": "CC2D2A",
  "term_id": "GO:1904491",
  "gene_name": "Coiled-coil and C2 domain-containing protein 2A"
}